(-)-lariciresinol catabolic process [GO:1902128] (biological process) References: PMID:15949826, PMID:9872995 Sources: GOC:TermGenie Relationships: is a type of phenol-containing compound catabolic process [GO:0019336]; is a type of lignan catabolic process [GO:0046273] Also known as: (-)-lariciresinol breakdown, (-)-lariciresinol catabolism, (-)-lariciresinol degradation Definition: The chemical reactions and pathways resulting in the breakdown of (-)-lariciresinol.